{
  "term_id": "UNKNOWN:0001",
  "gene_name": "Normal mucosa of esophagus-specific gene 1 protein",
  "gene_symbol": "NMES1",
  "gene": "UniProtKB:Q9C002",
  "term_label": "Unknown molecular function"
}